{
  "gene_name": "Solute carrier family 2, facilitated glucose transporter member 4",
  "term_id": "GO:0055056",
  "term_label": "D-glucose transmembrane transporter activity",
  "gene_symbol": "SLC2A4",
  "gene": "UniProtKB:P14672"
}